{
  "term_label": "axoneme",
  "gene_name": "Radial spoke head protein 4 homolog A",
  "gene_symbol": "RSPH4A",
  "gene": "UniProtKB:Q5TD94",
  "term_id": "GO:0005930"
}